{
  "term_id": "GO:0005886",
  "gene_name": "Olfactory receptor 2AE1",
  "gene": "UniProtKB:Q8NHA4",
  "gene_symbol": "OR2AE1",
  "term_label": "plasma membrane"
}